dATP(dGTP)-DNA purinetransferase activity [GO:0047839] (molecular function) Definition: Catalysis of the reaction: dATP + depurinated DNA = ribose triphosphate + DNA. Relationships: is a type of transferase activity, transferring nitrogenous groups [GO:0016769]; is a type of catalytic activity, acting on DNA [GO:0140097] Sources: EC:2.6.99.1 Also known as: dATP(dGTP)--DNA purine transferase activity, dATP(dGTP):depurinated-DNA purine transferase activity